{
  "gene_name": "RNA helicase Mov10l1",
  "term_id": "GO:0035194",
  "gene_symbol": "MOV10L1",
  "term_label": "regulatory ncRNA-mediated post-transcriptional gene silencing",
  "gene": "UniProtKB:Q9BXT6"
}